negative regulation of telomere capping [GO:1904354] (biological process) Subtypes: negative regulation of protection from non-homologous end joining at telomere [GO:1905765] Relationships: is a type of negative regulation of telomere maintenance [GO:0032205]; is a type of regulation of telomere capping [GO:1904353]; negatively regulates telomere capping [GO:0016233] References: PMID:23959892 Sources: GOC:BHF, GOC:BHF_telomere, GOC:TermGenie, GOC:nc, GO_REF:0000058 Also known as: down regulation of telomere capping, down regulation of telomere end protection, down-regulation of telomere capping, down-regulation of telomere end protection, downregulation of telomere capping, downregulation of telomere end protection, negative regulation of telomere end protection, inhibition of telomere capping, inhibition of telomere end protection Definition: Any process that stops, prevents or reduces the frequency, rate or extent of telomere capping.